{
  "gene_name": "Developmentally-regulated GTP-binding protein 1",
  "gene_symbol": "DRG1",
  "term_label": "cytoplasmic translation",
  "gene": "UniProtKB:Q9Y295",
  "term_id": "GO:0002181"
}